negative regulation of endothelial tube morphogenesis [GO:1905955] (biological process) References: PMID:25961718 Sources: GOC:BHF, GOC:BHF_miRNA, GOC:TermGenie, GOC:rph, GO_REF:0000058 Definition: Any process that stops, prevents or reduces the frequency, rate or extent of endothelial tube morphogenesis. Relationships: is a type of negative regulation of multicellular organismal process [GO:0051241]; is a type of regulation of endothelial tube morphogenesis [GO:1901509]; is a type of negative regulation of morphogenesis of an epithelium [GO:1905331]; negatively regulates endothelial tube morphogenesis [GO:0061154] Also known as: down regulation of endothelial tube morphogenesis, down-regulation of endothelial tube morphogenesis, downregulation of endothelial tube morphogenesis, inhibition of endothelial tube morphogenesis